{
  "term_id": "GO:0050911",
  "gene": "UniProtKB:A0A286YEU6",
  "term_label": "detection of chemical stimulus involved in sensory perception of smell",
  "gene_symbol": "A0A286YEU6",
  "gene_name": "Olfactory receptor family 1 subfamily R member 1 pseudogene"
}